{
  "term_id": "GO:0006893",
  "gene": "UniProtKB:Q6P1M3",
  "gene_name": "LLGL scribble cell polarity complex component 2",
  "term_label": "Golgi to plasma membrane transport",
  "gene_symbol": "LLGL2"
}